negative regulation of cardiocyte differentiation [GO:1905208] (biological process) Subtypes: negative regulation of cardioblast differentiation [GO:0051892], negative regulation of endocardial cushion cell differentiation [GO:0120076], negative regulation of cardiac cell fate specification [GO:2000044], GO:2000723, negative regulation of cardiac muscle cell differentiation [GO:2000726] Relationships: is a type of negative regulation of cell differentiation [GO:0045596]; is a type of negative regulation of multicellular organismal process [GO:0051241]; is a type of regulation of cardiocyte differentiation [GO:1905207]; negatively regulates cardiocyte differentiation [GO:0035051] Also known as: down regulation of cardiac cell differentiation, down regulation of cardiocyte differentiation, down regulation of heart cell differentiation, down-regulation of cardiac cell differentiation, down-regulation of cardiocyte differentiation, down-regulation of heart cell differentiation, downregulation of cardiac cell differentiation, downregulation of cardiocyte differentiation, downregulation of heart cell differentiation, negative regulation of cardiac cell differentiation, negative regulation of heart cell differentiation, inhibition of cardiac cell differentiation, inhibition of cardiocyte differentiation, inhibition of heart cell differentiation Definition: Any process that stops, prevents or reduces the frequency, rate or extent of cardiocyte differentiation. References: PMID:23069713 Sources: GOC:BHF, GOC:BHF_miRNA, GOC:TermGenie, GOC:bc, GO_REF:0000058